{
  "term_id": "GO:0000981",
  "gene": "UniProtKB:Q6P280",
  "term_label": "DNA-binding transcription factor activity, RNA polymerase II-specific",
  "gene_name": "Zinc finger protein 529",
  "gene_symbol": "ZNF529"
}